regulation of viral process [GO:0050792] (BP) Relationships: is a type of regulation of biological process [GO:0050789]; regulates viral process [GO:0016032] Definition: Any process that modulates the rate or extent of the viral life cycle, the set of processes by which a virus reproduces and spreads among hosts. Subtypes: regulation by virus of viral protein levels in host cell [GO:0046719], GO:0046782, positive regulation of viral process [GO:0048524], negative regulation of viral process [GO:0048525], regulation of viral budding via host ESCRT complex [GO:1903772], GO:1903900, regulation of viral translation [GO:1904971] Sources: GOC:go_curators, GOC:tb Also known as: regulation of viral reproduction